{
  "term_id": "UNKNOWN:0002",
  "gene": "UniProtKB:A0A494C086",
  "gene_name": "Putative speedy protein E21",
  "term_label": "Unknown biological process",
  "gene_symbol": "SPDYE21"
}